{
  "term_id": "GO:0019770",
  "gene_name": "Low affinity immunoglobulin gamma Fc region receptor II-a",
  "gene_symbol": "FCGR2A",
  "gene": "UniProtKB:P12318",
  "term_label": "IgG receptor activity"
}